{
  "gene": "UniProtKB:P02655",
  "gene_symbol": "APOC2",
  "gene_name": "Apolipoprotein C-II",
  "term_id": "GO:0034382",
  "term_label": "chylomicron remnant clearance"
}